{
  "gene": "UniProtKB:Q8WW12",
  "gene_name": "PEST proteolytic signal-containing nuclear protein",
  "term_label": "proteasome-mediated ubiquitin-dependent protein catabolic process",
  "term_id": "GO:0043161",
  "gene_symbol": "PCNP"
}